{
  "gene_symbol": "LINC00615",
  "gene": "UniProtKB:Q96LM1",
  "term_id": "UNKNOWN:0003",
  "term_label": "Unknown cellular component",
  "gene_name": "Putative uncharacterized protein encoded by LINC00615"
}